{
  "gene_name": "Putative ATP-dependent RNA helicase DHX57",
  "gene": "UniProtKB:Q6P158",
  "term_id": "GO:0004386",
  "gene_symbol": "DHX57",
  "term_label": "helicase activity"
}